regulation of appetite [GO:0032098] (biological process) Also known as: regulation of hunger Subtypes: negative regulation of appetite [GO:0032099], positive regulation of appetite [GO:0032100] Relationships: is a type of GO:0065008; is part of response to nutrient levels [GO:0031667] Definition: Any process which modulates appetite, the desire or physical craving for food. Sources: GOC:add